{
  "term_label": "Unknown molecular function",
  "gene_name": "Putative inactive cytochrome P450 2G1",
  "gene": "UniProtKB:Q6ZSU1",
  "gene_symbol": "CYP2G1P",
  "term_id": "UNKNOWN:0001"
}